{
  "gene": "UniProtKB:A0A075B6W2",
  "gene_symbol": "TRAJ52",
  "term_id": "UNKNOWN:0002",
  "term_label": "Unknown biological process",
  "gene_name": "T cell receptor alpha joining 52 (Fragment)"
}